{
  "gene_name": "Transmembrane protein 101",
  "term_id": "UNKNOWN:0003",
  "gene": "UniProtKB:Q96IK0",
  "term_label": "Unknown cellular component",
  "gene_symbol": "TMEM101"
}